{
  "gene": "UniProtKB:Q8N729",
  "term_id": "GO:0007631",
  "gene_symbol": "NPW",
  "gene_name": "Neuropeptide W",
  "term_label": "feeding behavior"
}